progesterone receptor signaling pathway [GO:0050847] (biological process) Definition: A nuclear receptor-mediated signaling pathway initiated by a progesterone binding to an intracellular receptor of the nuclear receptor protein family, and ending with regulation of a downstream cellular process, e.g. transcription. References: PMID:14744870 Also known as: intracellular progesterone receptor signaling pathway, nuclear receptor-mediated progesterone signaling pathway, progesterone receptor signalling pathway Relationships: is a type of nuclear receptor-mediated steroid hormone signaling pathway [GO:0030518]